{
  "gene": "UniProtKB:Q9Y6D6",
  "gene_name": "Brefeldin A-inhibited guanine nucleotide-exchange protein 1",
  "term_id": "GO:0005802",
  "term_label": "trans-Golgi network",
  "gene_symbol": "ARFGEF1"
}